{
  "gene_name": "Sphingosine-1-phosphate phosphatase 2",
  "term_id": "GO:0046839",
  "gene_symbol": "SGPP2",
  "gene": "UniProtKB:Q8IWX5",
  "term_label": "phospholipid dephosphorylation"
}